postsynaptic spectrin-associated cytoskeleton [GO:0099189] (cellular component) References: PMID:28576936 Sources: GOC:dos Definition: The portion of the spectrin-associated cytoskeleton contained within the postsynapse. Relationships: is a type of spectrin-associated cytoskeleton [GO:0014731]; is a type of postsynaptic cytoskeleton [GO:0099571]